{
  "term_label": "positive regulation of fibrinolysis",
  "gene_symbol": "F11",
  "gene": "UniProtKB:P03951",
  "term_id": "GO:0051919",
  "gene_name": "Coagulation factor XI"
}